glucanosyltransferase activity [GO:0042123] (molecular function) Subtypes: 1,3-beta-glucanosyltransferase activity [GO:0042124] Sources: GOC:jl Definition: Catalysis of the splitting and linkage of glucan molecules, resulting in glucan chain elongation. Relationships: is a type of transferase activity [GO:0016740]